{
  "term_id": "GO:0042147",
  "gene": "UniProtKB:Q9P2D3",
  "term_label": "retrograde transport, endosome to Golgi",
  "gene_symbol": "HEATR5B",
  "gene_name": "HEAT repeat-containing protein 5B"
}